response to potassium ion [GO:0035864] (biological process) Sources: GOC:yaf Subtypes: GO:0035865 Relationships: is a type of response to metal ion [GO:0010038] Also known as: response to K+ ion, response to potassium Definition: Any process that results in a change in state or activity of a cell or an organism (in terms of movement, secretion, enzyme production, gene expression, etc.) as a result of a potassium ion stimulus.